regulation of abscisic acid biosynthetic process [GO:0010115] (biological process) Also known as: regulation of abscisic acid anabolism, regulation of abscisic acid biosynthesis, regulation of abscisic acid formation, regulation of abscisic acid synthesis Subtypes: positive regulation of abscisic acid biosynthetic process [GO:0010116], negative regulation of abscisic acid biosynthetic process [GO:0090359] Relationships: is_a regulation of isoprenoid metabolic process [GO:0019747]; is a type of GO:0046890; is a type of GO:1902930; regulates abscisic acid biosynthetic process [GO:0009688] Definition: Any process that modulates the frequency, rate or extent of the chemical reactions and pathways resulting in the formation of abscisic acid. Sources: GOC:sm